{
  "term_label": "Unknown cellular component",
  "term_id": "UNKNOWN:0003",
  "gene_symbol": "OR9A1P",
  "gene": "UniProtKB:Q8NGU1",
  "gene_name": "Olfactory receptor 9A1"
}